{
  "term_id": "GO:0005737",
  "gene": "UniProtKB:A6NKC9",
  "gene_name": "SH2 domain-containing protein 7",
  "term_label": "cytoplasm",
  "gene_symbol": "SH2D7"
}